{
  "gene_symbol": "TRIM64",
  "term_id": "GO:0005737",
  "gene_name": "Tripartite motif-containing protein 64",
  "gene": "UniProtKB:A6NGJ6",
  "term_label": "cytoplasm"
}